{
  "gene_name": "Septin-7",
  "term_id": "GO:0005940",
  "term_label": "septin ring",
  "gene": "UniProtKB:Q16181",
  "gene_symbol": "SEPTIN7"
}